N-methyltransferase activity [GO:0008170] (molecular function) Sources: GOC:ai Relationships: is a type of methyltransferase activity [GO:0008168] Subtypes: rRNA (adenine-N6,N6-)-dimethyltransferase activity [GO:0000179], phosphoethanolamine N-methyltransferase activity [GO:0000234], phosphatidyl-N-methylethanolamine N-methyltransferase activity [GO:0000773], GO:0004482, phenylethanolamine N-methyltransferase activity [GO:0004603], phosphatidylethanolamine N-methyltransferase activity [GO:0004608], GO:0008112, nicotinate N-methyltransferase activity [GO:0008938], rRNA (adenine-N6-)-methyltransferase activity [GO:0008988], rRNA (guanine-N1-)-methyltransferase activity [GO:0008989], rRNA (guanine-N2-)-methyltransferase activity [GO:0008990], GO:0016273, lysine N-methyltransferase activity [GO:0016278], tRNA (adenine-N6)-methyltransferase activity [GO:0016430], GO:0017174, protein-L-histidine N-tele-methyltransferase activity [GO:0018064], protein-glutamine N-methyltransferase activity [GO:0036009], histamine N-methyltransferase activity [GO:0046539], GO:0047147, methylamine-glutamate N-methyltransferase activity [GO:0047148], dimethylglycine N-methyltransferase activity [GO:0052729], GO:0052730, rRNA (uridine-N3-)-methyltransferase activity [GO:0070042], GO:0070043, GO:0071424, GO:0106370, tRNA (guanine(10)-N2)-dimethyltransferase activity [GO:0160101], tRNA (guanine(10)-N2)-methyltransferase activity [GO:0160102], tRNA (guanine(26)-N2/guanine(27)-N2)-dimethyltransferase activity [GO:0160103], tRNA (guanine(26)-N2)-dimethyltransferase activity [GO:0160104], tRNA (guanine(6)-N2)-methyltransferase activity [GO:0160117], tRNA (guanine(7)-N2)-methyltransferase activity [GO:0160118], tRNA (guanine(27)-N2)-dimethyltransferase activity [GO:0160248] Definition: Catalysis of the transfer of a methyl group to the nitrogen atom of an acceptor molecule.